{
  "term_id": "GO:0005829",
  "term_label": "cytosol",
  "gene_name": "Elongator complex protein 5",
  "gene": "UniProtKB:Q8TE02",
  "gene_symbol": "ELP5"
}